{
  "term_id": "GO:0005789",
  "gene_name": "E3 ubiquitin-protein ligase RNF186",
  "gene_symbol": "RNF186",
  "term_label": "endoplasmic reticulum membrane",
  "gene": "UniProtKB:Q9NXI6"
}